{
  "term_id": "GO:1902490",
  "gene": "UniProtKB:B4DZS4",
  "gene_symbol": "TCP11X1",
  "gene_name": "T-complex protein 11 X-linked protein 1",
  "term_label": "regulation of sperm capacitation"
}